{
  "gene_name": "D-dopachrome decarboxylase",
  "gene_symbol": "DDT",
  "term_label": "phenylpyruvate tautomerase activity",
  "term_id": "GO:0050178",
  "gene": "UniProtKB:P30046"
}